cell swimming [GO:0071975] (BP) Also known as: cell swimming motility References: PMID:18461074 Definition: Cell motility that results in the smooth movement of a cell through a liquid medium. Relationships: is a type of cell motility [GO:0048870] Subtypes: GO:0071977, GO:0071979